spermidine catabolic process [GO:0046203] (biological process) Definition: The chemical reactions and pathways resulting in the breakdown of spermidine, N-(3-aminopropyl)-1,4-diaminobutane. Sources: GOC:ai Relationships: is_a polyamine catabolic process [GO:0006598]; is a type of spermidine metabolic process [GO:0008216] Also known as: spermidine breakdown, spermidine catabolism, spermidine degradation